{
  "gene": "UniProtKB:Q9HC44",
  "term_label": "DNA-binding transcription factor activity",
  "gene_symbol": "GPBP1L1",
  "term_id": "GO:0003700",
  "gene_name": "Vasculin-like protein 1"
}